{
  "gene_name": "Protein arginine N-methyltransferase 1",
  "gene_symbol": "PRMT1",
  "term_label": "protein-arginine omega-N asymmetric methyltransferase activity",
  "gene": "UniProtKB:Q99873",
  "term_id": "GO:0035242"
}